{
  "gene": "UniProtKB:Q6ZYL4",
  "gene_symbol": "GTF2H5",
  "gene_name": "General transcription factor IIH subunit 5",
  "term_id": "GO:0006366",
  "term_label": "transcription by RNA polymerase II"
}